{
  "gene": "UniProtKB:Q5HYW3",
  "term_id": "UNKNOWN:0003",
  "gene_symbol": "RTL5",
  "gene_name": "Retrotransposon Gag-like protein 5",
  "term_label": "Unknown cellular component"
}